{
  "gene_symbol": "LDHC",
  "gene": "UniProtKB:P07864",
  "term_label": "lactate metabolic process",
  "gene_name": "L-lactate dehydrogenase C chain",
  "term_id": "GO:0006089"
}